{
  "gene_symbol": "ADRA1A",
  "term_id": "GO:0007267",
  "gene_name": "Alpha-1A adrenergic receptor",
  "term_label": "cell-cell signaling",
  "gene": "UniProtKB:P35348"
}